{
  "term_id": "GO:0005525",
  "gene_symbol": "RAB34",
  "gene_name": "Ras-related protein Rab-34",
  "term_label": "GTP binding",
  "gene": "UniProtKB:Q9BZG1"
}